{
  "term_label": "endoplasmic reticulum",
  "term_id": "GO:0005783",
  "gene_symbol": "TMEM151A",
  "gene": "UniProtKB:Q8N4L1",
  "gene_name": "Transmembrane protein 151A"
}